{
  "gene_symbol": "SLC12A4",
  "gene": "UniProtKB:Q9UP95",
  "term_id": "GO:0007268",
  "term_label": "chemical synaptic transmission",
  "gene_name": "Solute carrier family 12 member 4"
}